{
  "term_label": "Unknown cellular component",
  "gene_name": "PDZ domain-containing protein GIPC2",
  "term_id": "UNKNOWN:0003",
  "gene_symbol": "GIPC2",
  "gene": "UniProtKB:Q8TF65"
}